{
  "gene_symbol": "H2BC11",
  "gene": "UniProtKB:P06899",
  "gene_name": "Histone H2B type 1-J",
  "term_label": "innate immune response in mucosa",
  "term_id": "GO:0002227"
}